{
  "term_label": "plasma membrane",
  "gene_name": "Ephrin type-A receptor 4",
  "gene": "UniProtKB:P54764",
  "gene_symbol": "EPHA4",
  "term_id": "GO:0005886"
}